{
  "term_label": "actin cytoskeleton organization",
  "gene": "UniProtKB:P53667",
  "term_id": "GO:0030036",
  "gene_name": "LIM domain kinase 1",
  "gene_symbol": "LIMK1"
}